{
  "term_id": "UNKNOWN:0001",
  "gene": "UniProtKB:A0A075B6W4",
  "gene_name": "T cell receptor alpha joining 46 (Fragment)",
  "gene_symbol": "TRAJ46",
  "term_label": "Unknown molecular function"
}